{
  "gene": "UniProtKB:Q07021",
  "gene_symbol": "C1QBP",
  "term_label": "regulation of complement activation",
  "term_id": "GO:0030449",
  "gene_name": "Complement component 1 Q subcomponent-binding protein, mitochondrial"
}